{
  "term_id": "GO:0005886",
  "gene_name": "Chondroadherin",
  "term_label": "plasma membrane",
  "gene": "UniProtKB:O15335",
  "gene_symbol": "CHAD"
}